{
  "gene_name": "Protocadherin alpha-5",
  "gene": "UniProtKB:Q9Y5H7",
  "term_label": "cell adhesion",
  "term_id": "GO:0007155",
  "gene_symbol": "PCDHA5"
}